{
  "term_id": "GO:0031530",
  "term_label": "gonadotropin-releasing hormone receptor binding",
  "gene_name": "Progonadoliberin-1",
  "gene": "UniProtKB:P01148",
  "gene_symbol": "GNRH1"
}